dosage compensation complex assembly [GO:0042714] (biological process) Definition: The aggregation, arrangement and bonding together of proteins on DNA or RNA to form the complex that mediates dosage compensation on one or more X chromosomes. References: PMID:11102361, PMID:12672493 Sources: GOC:jl Relationships: is a type of protein-containing complex assembly [GO:0065003]; is part of sex-chromosome dosage compensation [GO:0007549]